{
  "gene_name": "Immunoglobulin lambda variable 1-40",
  "term_id": "UNKNOWN:0001",
  "gene": "UniProtKB:P01703",
  "term_label": "Unknown molecular function",
  "gene_symbol": "IGLV1-40"
}